macropinosome [GO:0044354] (cellular component) Relationships: is a type of GO:0044352 References: PMID:14732047 Definition: A membrane-bounded, uncoated intracellular vesicle formed by the process of macropinocytosis.